{
  "term_label": "RNA binding",
  "gene_symbol": "RO60",
  "gene_name": "RNA-binding protein RO60",
  "gene": "UniProtKB:P10155",
  "term_id": "GO:0003723"
}